alpha-1,3-mannosylglycoprotein 4-beta-N-acetylglucosaminyltransferase activity [GO:0008454] (molecular function) Definition: Catalysis of the reaction: UDP-N-acetyl-D-glucosamine + (N-acetyl-beta-D-glucosaminyl-1,2)-alpha-D-mannosyl-1,3-(beta-N-acetyl-D-glucosaminyl-1,2-alpha-D-mannosyl-1,6)-beta-D-mannosyl-R = UDP + N-acetyl-beta-D-glucosaminyl-1,4-(N-acetyl-D-glucosaminyl-1,2)-alpha-D-mannosyl-1,3-(beta-N-acetyl-D-glucosaminyl-1,2-alpha-D-mannosyl-1,6)-beta-D-mannosyl-R. Sources: EC:2.4.1.145 Also known as: alpha-1,3-mannosylglycoprotein beta-1,4-N-acetylglucosaminyltransferase activity, GnTIV activity, N-acetylglucosaminyltransferase IV activity, N-glycosyl-oligosaccharide-glycoprotein N-acetylglucosaminyltransferase IV activity, UDP-N-acetyl-D-glucosamine:3-[2-(N-acetyl-beta-D-glucosaminyl)-alpha-D-mannosyl]-glycoprotein 4-beta-N-acetyl-D-glucosaminyltransferase activity, alpha-1,3-mannosyl-glycoprotein 4-beta-N-acetylglucosaminyltransferase activity, beta-acetylglucosaminyltransferase IV activity, uridine diphosphoacetylglucosamine-glycopeptide beta-4-acetylglucosaminyltransferase IV activity, uridine diphosphoacetylglucosamine-glycopeptide beta4-acetylglucosaminyltransferase IV Relationships: is a type of acetylglucosaminyltransferase activity [GO:0008375]; is a type of catalytic activity, acting on a glycoprotein [GO:0140103]